{
  "gene_symbol": "RMI1",
  "gene": "UniProtKB:Q9H9A7",
  "gene_name": "RecQ-mediated genome instability protein 1",
  "term_label": "double-strand break repair via homologous recombination",
  "term_id": "GO:0000724"
}